negative regulation of positive chemotaxis to cAMP [GO:0061123] (biological process) Definition: Any process that decreases the rate, frequency, or extent of directed movement of a motile cell or organism up a concentration gradient of 3',5'-cAMP. Subtypes: negative regulation of positive chemotaxis to cAMP by chlorinated alkylphenone [GO:0061125] Sources: GOC:dph Relationships: is a type of negative regulation of positive chemotaxis [GO:0050928]; is a type of regulation of positive chemotaxis to cAMP [GO:0061118]; negatively regulates chemotaxis to cAMP [GO:0043327]